{
  "gene_symbol": "BARX1",
  "term_id": "GO:0000977",
  "gene_name": "Homeobox protein BarH-like 1",
  "gene": "UniProtKB:Q9HBU1",
  "term_label": "RNA polymerase II transcription regulatory region sequence-specific DNA binding"
}